{
  "gene": "UniProtKB:Q9Y312",
  "gene_name": "Protein AAR2 homolog",
  "term_id": "GO:0000244",
  "gene_symbol": "AAR2",
  "term_label": "spliceosomal tri-snRNP complex assembly"
}